pectin catabolic process [GO:0045490] (biological process) Also known as: pectin breakdown, pectin catabolism, pectin degradation Definition: The chemical reactions and pathways resulting in the breakdown of pectin, a polymer containing a backbone of alpha-1,4-linked D-galacturonic acid residues. Regulation: regulated by GO:2001003; negatively regulated by GO:2001004; positively regulated by GO:2001005 Subtypes: anaerobic pectin catabolic process [GO:1990489] References: PMID:11931668 Sources: GOC:go_curators Relationships: is a type of polysaccharide catabolic process [GO:0000272]; is a type of pectin metabolic process [GO:0045488]